{
  "gene_symbol": "IL15",
  "gene_name": "Interleukin-15",
  "term_id": "GO:0005125",
  "gene": "UniProtKB:P40933",
  "term_label": "cytokine activity"
}